{
  "gene_name": "GTP-binding protein Rhes",
  "gene": "UniProtKB:Q96D21",
  "term_id": "UNKNOWN:0003",
  "term_label": "Unknown cellular component",
  "gene_symbol": "RASD2"
}